rRNA (guanine) methyltransferase activity [GO:0016435] (molecular function) Relationships: is a type of rRNA methyltransferase activity [GO:0008649] Subtypes: rRNA (guanine-N1-)-methyltransferase activity [GO:0008989], rRNA (guanine-N2-)-methyltransferase activity [GO:0008990], rRNA (guanosine-2'-O-)-methyltransferase activity [GO:0070039], rRNA (guanine-N7-)-methyltransferase activity [GO:0070043] Definition: Catalysis of the reaction: S-adenosyl-L-methionine + rRNA = S-adenosyl-L-homocysteine + rRNA containing methylguanine. Sources: GOC:curators